{
  "gene": "UniProtKB:Q5XUX1",
  "term_label": "Unknown cellular component",
  "term_id": "UNKNOWN:0003",
  "gene_symbol": "FBXW9",
  "gene_name": "F-box_WD repeat-containing protein 9"
}